{
  "gene_name": "Heat shock factor protein 2",
  "term_label": "nucleus",
  "gene": "UniProtKB:Q03933",
  "gene_symbol": "HSF2",
  "term_id": "GO:0005634"
}